{
  "term_id": "UNKNOWN:0001",
  "gene_symbol": "NDUFAF8",
  "gene_name": "NADH dehydrogenase [ubiquinone] 1 alpha subcomplex assembly factor 8",
  "gene": "UniProtKB:A1L188",
  "term_label": "Unknown molecular function"
}